negative regulation of mitotic spindle elongation [GO:1902845] (biological process) References: PMID:23087209 Sources: GOC:TermGenie, GO_REF:0000058 Definition: Any process that stops, prevents or reduces the frequency, rate or extent of mitotic spindle elongation. Subtypes: negative regulation of mitotic spindle elongation (spindle phase three) [GO:0110163] Relationships: is a type of negative regulation of cell cycle process [GO:0010948]; is a type of regulation of mitotic spindle elongation [GO:0032888]; RO_0002212 mitotic spindle elongation [GO:0000022] Also known as: down regulation of mitotic spindle elongation, down regulation of spindle elongation during mitosis, down-regulation of mitotic spindle elongation, down-regulation of spindle elongation during mitosis, downregulation of mitotic spindle elongation, downregulation of spindle elongation during mitosis, negative regulation of spindle elongation during mitosis, inhibition of mitotic spindle elongation, inhibition of spindle elongation during mitosis